{
  "term_id": "UNKNOWN:0003",
  "term_label": "Unknown cellular component",
  "gene": "UniProtKB:O75884",
  "gene_symbol": "RBBP9",
  "gene_name": "Serine hydrolase RBBP9"
}